{
  "gene_name": "Putative zinc finger protein 542",
  "gene_symbol": "ZNF542P",
  "gene": "UniProtKB:Q5EBM4",
  "term_label": "Unknown molecular function",
  "term_id": "UNKNOWN:0001"
}